{
  "term_label": "glucose 6-phosphate metabolic process",
  "gene_name": "Hexokinase-1",
  "gene_symbol": "HK1",
  "gene": "UniProtKB:P19367",
  "term_id": "GO:0051156"
}